{
  "gene_name": "Vacuolar protein sorting-associated protein 72 homolog",
  "gene_symbol": "VPS72",
  "term_label": "histone chaperone activity",
  "term_id": "GO:0140713",
  "gene": "UniProtKB:Q15906"
}